histone H4K5 acetyltransferase activity [GO:0043995] (MF) Also known as: histone acetylase activity (H4-K5 specific), histone acetyltransferase activity (H4-K5 specific), histone lysine N-acetyltransferase activity (H4-K5 specific) Relationships: is a type of histone H4 acetyltransferase activity [GO:0010485] Note: Note that the residue position corresponds to the canonical human H4 histone (UniProtKB:P02309); this residue is conserved across all eukaryotes. Note that the initiation methionine is cleaved, so the first residue is S1. Definition: Catalysis of the reaction: acetyl-CoA + histone H4 L-lysine (position 5) = CoA + histone H4 N6-acetyl-L-lysine (position 5). References: PMID:18552846, PMID:19056256